{
  "gene": "UniProtKB:Q8NGQ4",
  "term_label": "olfactory receptor activity",
  "gene_name": "Olfactory receptor 10Q1",
  "term_id": "GO:0004984",
  "gene_symbol": "OR10Q1"
}